{
  "term_label": "neutrophil aggregation",
  "term_id": "GO:0070488",
  "gene_name": "Protein S100-A8",
  "gene": "UniProtKB:P05109",
  "gene_symbol": "S100A8"
}